{
  "term_id": "GO:0005886",
  "term_label": "plasma membrane",
  "gene_name": "Transient receptor potential cation channel subfamily M member 8",
  "gene": "UniProtKB:Q7Z2W7",
  "gene_symbol": "TRPM8"
}